{
  "term_id": "GO:0061028",
  "term_label": "establishment of endothelial barrier",
  "gene_name": "Protein phosphatase 1 regulatory inhibitor subunit 16B",
  "gene_symbol": "PPP1R16B",
  "gene": "UniProtKB:Q96T49"
}